{
  "term_label": "nuclear import signal receptor activity",
  "gene_symbol": "KPNA3",
  "gene": "UniProtKB:O00505",
  "gene_name": "Importin subunit alpha-4",
  "term_id": "GO:0061608"
}